{
  "gene": "UniProtKB:Q96I13",
  "gene_name": "Protein ABHD8",
  "term_label": "carboxylic ester hydrolase activity",
  "term_id": "GO:0052689",
  "gene_symbol": "ABHD8"
}